{
  "gene_name": "TBC1 domain family member 24",
  "gene": "UniProtKB:Q9ULP9",
  "gene_symbol": "TBC1D24",
  "term_label": "plasma membrane",
  "term_id": "GO:0005886"
}